glycerophospholipid flippase activity [GO:0140333] (molecular function) Subtypes: phosphatidylethanolamine flippase activity [GO:0090555], GO:0140345, phosphatidylserine flippase activity [GO:0140346], N-retinylidene-phosphatidylethanolamine flippase activity [GO:0140347], lysophosphatidylcholine flippase activity [GO:0140348], lysophosphatidylserine flippase activity [GO:0180013] References: PMID:26212235 Definition: Catalysis of the movement of a glycerophospholipid from the exoplasmic to the cytosolic leaflet of a membrane, using energy from the hydrolysis of ATP. Also known as: glycerophospholipid flippase activity (exoplasmic to cytosolic leaflet) Relationships: is a type of phospholipid transporter activity [GO:0005548]; is a type of flippase activity [GO:0140327]